{
  "term_id": "GO:0008113",
  "gene": "UniProtKB:Q9UJ68",
  "gene_symbol": "MSRA",
  "term_label": "peptide-methionine (S)-S-oxide reductase activity",
  "gene_name": "Mitochondrial peptide methionine sulfoxide reductase"
}